perforin production [GO:0035944] (biological process) Relationships: is a type of GO:0002440 Definition: The appearance of a perforin protein due to biosynthesis or secretion following a cellular stimulus, resulting in an increase in its intracellular or extracellular levels. Sources: GOC:rv Note: Note that this term is in the subset of terms that should not be used for direct gene product annotation. Instead, select one of the 'regulation' children terms.